{
  "gene_name": "Exocyst complex component 4",
  "term_id": "GO:0006887",
  "term_label": "exocytosis",
  "gene": "UniProtKB:Q96A65",
  "gene_symbol": "EXOC4"
}